{
  "gene_symbol": "OR52D1",
  "term_id": "GO:0005886",
  "gene_name": "Olfactory receptor 52D1",
  "term_label": "plasma membrane",
  "gene": "UniProtKB:Q9H346"
}